{
  "gene_name": "Vesicular glutamate transporter 1",
  "gene_symbol": "SLC17A7",
  "term_label": "synaptic transmission, glutamatergic",
  "term_id": "GO:0035249",
  "gene": "UniProtKB:Q9P2U7"
}